{
  "gene": "UniProtKB:Q9H4L7",
  "term_label": "chromatin",
  "term_id": "GO:0000785",
  "gene_symbol": "SMARCAD1",
  "gene_name": "SWI_SNF-related matrix-associated actin-dependent regulator of chromatin subfamily A containing DEAD_H box 1"
}